negative regulation of RIG-I signaling pathway [GO:0039536] (biological process) Definition: Any process that stops, prevents, or reduces the frequency, rate or extent of the RIG-I signaling pathway. Also known as: negative regulation of DDX58 signaling pathway, negative regulation of RIG-I signalling pathway, negative regulation of retinoic acid inducible gene I signaling pathway Relationships: is_a GO:0039532; is a type of regulation of RIG-I signaling pathway [GO:0039535]; negatively regulates RIG-I signaling pathway [GO:0039529] Sources: GOC:bf, GOC:jl